{
  "gene_name": "Signal transducer and activator of transcription 6",
  "gene": "UniProtKB:P42226",
  "gene_symbol": "STAT6",
  "term_label": "regulation of cell population proliferation",
  "term_id": "GO:0042127"
}